{
  "term_label": "positive regulation of cytosolic calcium ion concentration",
  "gene_symbol": "CCR2",
  "term_id": "GO:0007204",
  "gene_name": "C-C chemokine receptor type 2",
  "gene": "UniProtKB:P41597"
}